{
  "term_id": "GO:0002218",
  "term_label": "activation of innate immune response",
  "gene_name": "Stimulator of interferon genes protein",
  "gene": "UniProtKB:Q86WV6",
  "gene_symbol": "STING1"
}